{
  "gene_name": "Gelsolin",
  "term_label": "barbed-end actin filament capping",
  "gene": "UniProtKB:P06396",
  "gene_symbol": "GSN",
  "term_id": "GO:0051016"
}